{
  "term_id": "UNKNOWN:0001",
  "gene": "UniProtKB:Q92777",
  "term_label": "Unknown molecular function",
  "gene_symbol": "SYN2",
  "gene_name": "Synapsin-2"
}